myosin-light-chain-phosphatase activity [GO:0050115] (molecular function) Definition: Catalysis of the reaction: myosin light-chain phosphate + H2O = myosin light chain + phosphate. Relationships: is a type of GO:0004721 Sources: EC:3.1.3.53, MetaCyc:MYOSIN-LIGHT-CHAIN-PHOSPHATASE-RXN Also known as: [Myosin light-chain]-phosphatase activity, myosin light chain kinase phosphatase activity, myosin light-chain kinase phosphatase activity, myosin-light-chain phosphatase activity, myosin-light-chain-phosphate phosphohydrolase activity, protein phosphatase 2A